{
  "term_id": "GO:0000981",
  "gene_symbol": "RHOXF2",
  "gene": "UniProtKB:Q9BQY4",
  "gene_name": "Rhox homeobox family member 2",
  "term_label": "DNA-binding transcription factor activity, RNA polymerase II-specific"
}